{
  "gene_name": "Corticotropin-releasing factor-binding protein",
  "gene": "UniProtKB:P24387",
  "term_label": "corticotropin-releasing hormone binding",
  "gene_symbol": "CRHBP",
  "term_id": "GO:0051424"
}